cellular response to biotin [GO:0071296] (biological process) Also known as: cellular response to Bios IIB, cellular response to coenzyme R, cellular response to vitamin B7, cellular response to vitamin H Sources: GOC:mah Relationships: is a type of response to biotin [GO:0070781]; is a type of cellular response to vitamin [GO:0071295]; is a type of cellular response to nitrogen compound [GO:1901699]; is a type of cellular response to oxygen-containing compound [GO:1901701] Definition: Any process that results in a change in state or activity of a cell (in terms of movement, secretion, enzyme production, gene expression, etc.) as a result of a biotin stimulus.